{
  "gene": "UniProtKB:Q7Z2Y8",
  "gene_symbol": "GVINP1",
  "gene_name": "Interferon-induced very large GTPase 1",
  "term_label": "Unknown molecular function",
  "term_id": "UNKNOWN:0001"
}